vacuolar calcium ion homeostasis [GO:0007036] (biological process) Definition: Any process involved in the maintenance of an internal steady state of calcium ions in the vacuole or between a vacuole and its surroundings. Sources: GOC:ai, GOC:mah Relationships: is a type of intracellular calcium ion homeostasis [GO:0006874]; occurs in vacuole [GO:0005773]